{
  "gene": "UniProtKB:Q8NCF5",
  "gene_name": "NFATC2-interacting protein",
  "term_id": "UNKNOWN:0003",
  "gene_symbol": "NFATC2IP",
  "term_label": "Unknown cellular component"
}